{
  "gene": "UniProtKB:Q9UHQ4",
  "gene_symbol": "BCAP29",
  "term_label": "Unknown molecular function",
  "term_id": "UNKNOWN:0001",
  "gene_name": "B-cell receptor-associated protein 29"
}